{
  "term_id": "GO:0005615",
  "gene": "UniProtKB:P06858",
  "gene_symbol": "LPL",
  "term_label": "extracellular space",
  "gene_name": "Lipoprotein lipase"
}